{
  "gene_name": "CTP synthase 2",
  "term_label": "identical protein binding",
  "gene_symbol": "CTPS2",
  "term_id": "GO:0042802",
  "gene": "UniProtKB:Q9NRF8"
}